{
  "term_label": "protein tag activity",
  "gene": "UniProtKB:Q15843",
  "gene_name": "NEDD8",
  "term_id": "GO:0031386",
  "gene_symbol": "NEDD8"
}